{
  "gene": "UniProtKB:C9JLW8",
  "gene_symbol": "MCRIP1",
  "term_label": "Unknown molecular function",
  "term_id": "UNKNOWN:0001",
  "gene_name": "Mapk-regulated corepressor-interacting protein 1"
}